{
  "gene_symbol": "CEBPA",
  "gene_name": "CCAAT_enhancer-binding protein alpha",
  "gene": "UniProtKB:P49715",
  "term_label": "Unknown cellular component",
  "term_id": "UNKNOWN:0003"
}